{
  "gene_symbol": "SLC25A10",
  "gene_name": "Mitochondrial dicarboxylate carrier",
  "term_id": "GO:0015709",
  "term_label": "thiosulfate transport",
  "gene": "UniProtKB:Q9UBX3"
}